{
  "term_label": "Unknown molecular function",
  "gene_symbol": "TRDD1",
  "term_id": "UNKNOWN:0001",
  "gene_name": "T cell receptor delta diversity 1",
  "gene": "UniProtKB:P0DPR3"
}